{
  "gene_symbol": "KCNE4",
  "term_label": "potassium channel regulator activity",
  "gene": "UniProtKB:Q8WWG9",
  "term_id": "GO:0015459",
  "gene_name": "Potassium voltage-gated channel subfamily E member 4"
}